{
  "gene_name": "Insulin-like growth factor-binding protein 7",
  "term_id": "GO:0009966",
  "term_label": "regulation of signal transduction",
  "gene": "UniProtKB:Q16270",
  "gene_symbol": "IGFBP7"
}